negative regulation of Fc-gamma receptor signaling pathway involved in phagocytosis [GO:1905450] (biological process) Also known as: down regulation of Fc gamma receptor-dependent phagocytosis, down regulation of Fc-gamma receptor signaling pathway involved in phagocytosis, down regulation of Fc-gamma receptor signalling pathway involved in phagocytosis, down regulation of Fcgamma receptor-mediated phagocytosis, down regulation of IgG-mediated phagocytosis, down-regulation of Fc gamma receptor-dependent phagocytosis, down-regulation of Fc-gamma receptor signaling pathway involved in phagocytosis, down-regulation of Fc-gamma receptor signalling pathway involved in phagocytosis, down-regulation of Fcgamma receptor-mediated phagocytosis, down-regulation of IgG-mediated phagocytosis, downregulation of Fc gamma receptor-dependent phagocytosis, downregulation of Fc-gamma receptor signaling pathway involved in phagocytosis, downregulation of Fc-gamma receptor signalling pathway involved in phagocytosis, downregulation of Fcgamma receptor-mediated phagocytosis, downregulation of IgG-mediated phagocytosis, negative regulation of Fc gamma receptor-dependent phagocytosis, negative regulation of Fc-gamma receptor signalling pathway involved in phagocytosis, negative regulation of Fcgamma receptor-mediated phagocytosis, negative regulation of IgG-mediated phagocytosis, inhibition of Fc gamma receptor-dependent phagocytosis, inhibition of Fc-gamma receptor signaling pathway involved in phagocytosis, inhibition of Fc-gamma receptor signalling pathway involved in phagocytosis, inhibition of Fcgamma receptor-mediated phagocytosis, inhibition of IgG-mediated phagocytosis References: PMID:18832707 Sources: GOC:TermGenie, GO_REF:0000058 Definition: Any process that stops, prevents or reduces the frequency, rate or extent of Fc-gamma receptor signaling pathway involved in phagocytosis. Relationships: is a type of negative regulation of immune effector process [GO:0002698]; is a type of GO:0009968; is a type of negative regulation of phagocytosis [GO:0050765]; is a type of regulation of Fc-gamma receptor signaling pathway involved in phagocytosis [GO:1905449]; RO_0002212 GO:0038096